{
  "gene": "UniProtKB:Q5VW22",
  "term_id": "GO:0003924",
  "gene_name": "Arf-GAP with GTPase, ANK repeat and PH domain-containing protein 6",
  "gene_symbol": "AGAP6",
  "term_label": "GTPase activity"
}